{
  "gene": "UniProtKB:P08236",
  "term_id": "GO:0030207",
  "term_label": "chondroitin sulfate proteoglycan catabolic process",
  "gene_symbol": "GUSB",
  "gene_name": "Beta-glucuronidase"
}